{
  "term_label": "Unknown biological process",
  "gene_name": "Uncharacterized protein",
  "gene_symbol": "LOC114841035",
  "gene": "UniProtKB:A0A494C030",
  "term_id": "UNKNOWN:0002"
}